type 1E serotonin receptor binding [GO:0031824] (molecular function) Also known as: 5-hydroxytryptamine 1E receptor binding, type 1E serotonin receptor ligand Sources: GOC:mah, GOC:nln Definition: Binding to a type 1E serotonin receptor. Relationships: is a type of GO:0031821